negative regulation of thymocyte apoptotic process [GO:0070244] (biological process) Note: Note that a thymocyte is an immature T cell located in the thymus (CL:0000893). Definition: Any process that stops, prevents, or reduces the frequency, rate or extent of thymocyte death by apoptotic process. Also known as: down regulation of thymocyte apoptosis, down-regulation of thymocyte apoptosis, downregulation of thymocyte apoptosis, inhibition of thymocyte apoptosis, negative regulation of thymocyte apoptosis, negative regulation of immature T cell apoptosis Sources: GOC:add, GOC:mtg_apoptosis, ISBN:0781765196 Relationships: is a type of negative regulation of T cell apoptotic process [GO:0070233]; is a type of GO:0070243; negatively regulates GO:0070242